{
  "gene_symbol": "BRINP1",
  "term_id": "GO:0043025",
  "gene_name": "BMP_retinoic acid-inducible neural-specific protein 1",
  "term_label": "neuronal cell body",
  "gene": "UniProtKB:O60477"
}